{
  "gene": "UniProtKB:Q15116",
  "gene_symbol": "PDCD1",
  "term_label": "regulation of immune response",
  "gene_name": "Programmed cell death protein 1",
  "term_id": "GO:0050776"
}